{
  "term_label": "serine-type endopeptidase activity",
  "gene_symbol": "CELA3A",
  "term_id": "GO:0004252",
  "gene": "UniProtKB:P09093",
  "gene_name": "Chymotrypsin-like elastase family member 3A"
}